{
  "gene_symbol": "CACNA2D2",
  "term_id": "GO:0005891",
  "gene": "UniProtKB:Q9NY47",
  "term_label": "voltage-gated calcium channel complex",
  "gene_name": "Voltage-dependent calcium channel subunit alpha-2_delta-2"
}